{
  "gene_symbol": "CFAP74",
  "gene": "UniProtKB:Q9C0B2",
  "term_id": "UNKNOWN:0002",
  "gene_name": "Cilia- and flagella-associated protein 74",
  "term_label": "Unknown biological process"
}